{
  "gene_name": "Transforming acidic coiled-coil-containing protein 3",
  "term_id": "GO:0030953",
  "term_label": "astral microtubule organization",
  "gene": "UniProtKB:Q9Y6A5",
  "gene_symbol": "TACC3"
}